{
  "term_label": "integrin binding involved in cell-matrix adhesion",
  "gene_symbol": "MADCAM1",
  "gene_name": "Mucosal addressin cell adhesion molecule 1",
  "gene": "UniProtKB:Q13477",
  "term_id": "GO:0098640"
}